{
  "term_label": "RNA polymerase II cis-regulatory region sequence-specific DNA binding",
  "gene_name": "Highly divergent homeobox",
  "gene_symbol": "HDX",
  "gene": "UniProtKB:Q7Z353",
  "term_id": "GO:0000978"
}